dhurrin biosynthetic process [GO:0010132] (biological process) Sources: GOC:pz Also known as: dhurrin anabolism, dhurrin biosynthesis, dhurrin formation, dhurrin synthesis Relationships: is a type of GO:0019756; is a type of beta-glucoside biosynthetic process [GO:1901806] Definition: The chemical reactions and pathways resulting in the formation of dhurrin, a cyanogenic glucoside which functions as a plant defense compound.